{
  "gene": "UniProtKB:Q8TE67",
  "term_id": "GO:0035023",
  "gene_name": "Epidermal growth factor receptor kinase substrate 8-like protein 3",
  "term_label": "regulation of Rho protein signal transduction",
  "gene_symbol": "EPS8L3"
}